tRNA (cytidine) methyltransferase activity [GO:0016427] (molecular function) Definition: Catalysis of the reaction: S-adenosyl-L-methionine + tRNA = S-adenosyl-L-homocysteine + tRNA containing methylcytosine. Sources: GOC:go-curators Also known as: tRNA (cytosine) methyltransferase activity Relationships: is a type of tRNA methyltransferase activity [GO:0008175]; is a type of S-adenosylmethionine-dependent methyltransferase activity [GO:0008757] Subtypes: tRNA (cytidine-5-)-methyltransferase activity [GO:0016428], tRNA (cytidine-3-)-methyltransferase activity [GO:0052735], tRNA (cytidine(56)-2'-O)-methyltransferase activity [GO:0106059], GO:0106339, tRNA (cytidine(34)-2'-O)-methyltransferase activity [GO:0141098], tRNA (cytidine(32)/uridine(32)-2'-O)-methyltransferase activity [GO:0160206]